{
  "term_label": "axonal transport of mitochondrion",
  "gene_symbol": "ARMCX2",
  "term_id": "GO:0019896",
  "gene_name": "Armadillo repeat-containing X-linked protein 2",
  "gene": "UniProtKB:Q7L311"
}